proximal convoluted tubule segment 1 development [GO:0072031] (biological process) Subtypes: metanephric proximal convoluted tubule segment 1 development [GO:0072231] Definition: The process whose specific outcome is the progression of the S1 portion of the proximal convoluted tubule over time, from its formation to the mature structure. The S1 portion is the initial portion of the proximal convoluted tubule and is responsible for avid reabsorption of water and solutes. Also known as: S1 development Relationships: is a type of tube development [GO:0035295]; is part of proximal convoluted tubule development [GO:0072019] Sources: GOC:mtg_kidney_jan10, MA:0002612